{
  "term_id": "UNKNOWN:0001",
  "gene": "UniProtKB:Q8NCR9",
  "gene_name": "Clarin-3",
  "gene_symbol": "CLRN3",
  "term_label": "Unknown molecular function"
}